histone octamer slider activity [GO:0140751] (molecular function) Definition: A chromatin remodeler activity that slides core histone octamers along chromosomal DNA. References: PMID:10466730 Also known as: histone octamer sliding activity Note: This activity is mediated by at least three subfamilies of the SNF2 remodellers, namely the bromodomain domain, the chromodomain containing and the imitation switch subfamilies. Relationships: is a type of ATP-dependent chromatin remodeler activity [GO:0140658] Subtypes: GO:0140750